{
  "gene_name": "Uncharacterized protein KIAA1614",
  "gene": "UniProtKB:Q5VZ46",
  "gene_symbol": "KIAA1614",
  "term_id": "GO:0005938",
  "term_label": "cell cortex"
}